{
  "gene_symbol": "SDK1",
  "term_label": "synapse assembly",
  "gene_name": "Protein sidekick-1",
  "gene": "UniProtKB:Q7Z5N4",
  "term_id": "GO:0007416"
}